{
  "term_label": "Unknown molecular function",
  "gene_symbol": "TNFSF8",
  "gene": "UniProtKB:P32971",
  "term_id": "UNKNOWN:0001",
  "gene_name": "Tumor necrosis factor ligand superfamily member 8"
}